{
  "gene_name": "Zinc finger protein 540",
  "gene_symbol": "ZNF540",
  "gene": "UniProtKB:Q8NDQ6",
  "term_id": "GO:0005634",
  "term_label": "nucleus"
}